{
  "gene_name": "Neurofilament medium polypeptide",
  "term_label": "structural constituent of cytoskeleton",
  "gene": "UniProtKB:P07197",
  "term_id": "GO:0005200",
  "gene_symbol": "NEFM"
}